{
  "gene": "UniProtKB:Q15375",
  "term_label": "ephrin receptor signaling pathway",
  "gene_name": "Ephrin type-A receptor 7",
  "gene_symbol": "EPHA7",
  "term_id": "GO:0048013"
}